{
  "term_label": "cellular response to lipopolysaccharide",
  "gene": "UniProtKB:Q9NRJ3",
  "term_id": "GO:0071222",
  "gene_symbol": "CCL28",
  "gene_name": "C-C motif chemokine 28"
}